polarisome [GO:0000133] (cellular component) Relationships: is a type of protein-containing complex [GO:0032991]; is part of GO:0005938; is part of GO:0030427 Subtypes: cellular bud neck polarisome [GO:0031560], GO:0031561, GO:0031562, mating projection tip polarisome [GO:0031563] References: PMID:14734532, PMID:14998522, PMID:9632790 Definition: Protein complex that plays a role in determining cell polarity by directing the localized assembly of actin filaments at polarization sites; in Saccharomyces the polarisome includes Bni1p, Spa2p, Pea2p, and Bud6p.